positive regulation of L-leucine biosynthetic process [GO:2001278] (biological process) Relationships: is a type of positive regulation of small molecule metabolic process [GO:0062013]; is a type of positive regulation of amino acid biosynthetic process [GO:2000284]; is a type of regulation of L-leucine biosynthetic process [GO:2001276]; positively regulates L-leucine biosynthetic process [GO:0009098] Definition: Any process that activates or increases the frequency, rate or extent of L-leucine biosynthetic process. Also known as: positive regulation of leucine biosynthetic process, positive regulation of L-leucine anabolism, positive regulation of L-leucine biosynthesis, positive regulation of L-leucine formation, positive regulation of L-leucine synthesis Sources: GOC:obol